{
  "gene": "UniProtKB:A0A087WSX0",
  "term_label": "immunoglobulin complex",
  "term_id": "GO:0019814",
  "gene_name": "Immunoglobulin lambda variable 5-45",
  "gene_symbol": "IGLV5-45"
}